{
  "gene": "UniProtKB:Q96EP5",
  "gene_symbol": "DAZAP1",
  "gene_name": "DAZ-associated protein 1",
  "term_id": "GO:0034046",
  "term_label": "poly(G) binding"
}